{
  "term_id": "GO:0005768",
  "gene_name": "Vacuolar protein sorting-associated protein 4B",
  "gene": "UniProtKB:O75351",
  "gene_symbol": "VPS4B",
  "term_label": "endosome"
}